 [owl#deprecated]